{
  "term_id": "GO:0005929",
  "gene_symbol": "DLEC1",
  "term_label": "cilium",
  "gene": "UniProtKB:Q9Y238",
  "gene_name": "Deleted in lung and esophageal cancer protein 1"
}